{
  "gene_symbol": "ACD",
  "term_label": "shelterin complex",
  "gene_name": "Adrenocortical dysplasia protein homolog",
  "term_id": "GO:0070187",
  "gene": "UniProtKB:Q96AP0"
}